{
  "term_id": "GO:0000981",
  "gene_symbol": "GATA3",
  "term_label": "DNA-binding transcription factor activity, RNA polymerase II-specific",
  "gene_name": "Trans-acting T-cell-specific transcription factor GATA-3",
  "gene": "UniProtKB:P23771"
}